{
  "term_id": "GO:0004371",
  "gene": "UniProtKB:Q3LXA3",
  "term_label": "glycerone kinase activity",
  "gene_symbol": "TKFC",
  "gene_name": "Triokinase_FMN cyclase"
}